calcium ion transport [GO:0006816] (biological process) Definition: The directed movement of calcium (Ca) ions into, out of or within a cell, or between cells, by means of some agent such as a transporter or pore. Subtypes: GO:0002115, Golgi calcium ion transport [GO:0032472], sarcoplasmic reticulum calcium ion transport [GO:0070296], GO:0070509, GO:0070588, GO:1901660, calcium ion import into cytosol [GO:1902656] Regulation: regulated by regulation of calcium ion transport [GO:0051924]; negatively regulated by negative regulation of calcium ion transport [GO:0051926]; positively regulated by GO:0051928 Also known as: calcium transport, mitochondrial sodium/calcium ion exchange, sodium:calcium exchange Sources: GOC:ai Relationships: is a type of GO:0030001